{
  "gene_symbol": "NAT9",
  "term_id": "GO:1901673",
  "gene_name": "Alpha_beta-tubulin-N-acetyltransferase 9",
  "gene": "UniProtKB:Q9BTE0",
  "term_label": "regulation of mitotic spindle assembly"
}